{
  "term_id": "GO:0042795",
  "term_label": "snRNA transcription by RNA polymerase II",
  "gene_name": "snRNA-activating protein complex subunit 4",
  "gene_symbol": "SNAPC4",
  "gene": "UniProtKB:Q5SXM2"
}